{
  "term_label": "external side of plasma membrane",
  "gene": "UniProtKB:Q86VB7",
  "gene_symbol": "CD163",
  "term_id": "GO:0009897",
  "gene_name": "Scavenger receptor cysteine-rich type 1 protein M130"
}